regulation of starch metabolic process [GO:2000904] (BP) Definition: Any process that modulates the frequency, rate or extent of starch metabolic process. Relationships: is a type of regulation of polysaccharide metabolic process [GO:0032881]; regulates GO:0005982 Also known as: regulation of starch metabolism Subtypes: GO:0010581, regulation of starch catabolic process [GO:2000881] Sources: GOC:obol